{
  "term_id": "UNKNOWN:0003",
  "gene_name": "T cell receptor delta diversity 1",
  "gene": "UniProtKB:P0DPR3",
  "term_label": "Unknown cellular component",
  "gene_symbol": "TRDD1"
}